{
  "gene_name": "Gamma-aminobutyric acid receptor-associated protein-like 1",
  "gene_symbol": "GABARAPL1",
  "term_id": "GO:0050811",
  "gene": "UniProtKB:Q9H0R8",
  "term_label": "GABA receptor binding"
}